{
  "term_id": "GO:0005856",
  "gene": "UniProtKB:O60662",
  "gene_symbol": "KLHL41",
  "gene_name": "Kelch-like protein 41",
  "term_label": "cytoskeleton"
}